{
  "gene_symbol": "HSP90AB2P",
  "gene": "UniProtKB:Q58FF8",
  "term_label": "ATP hydrolysis activity",
  "gene_name": "Putative heat shock protein HSP 90-beta 2",
  "term_id": "GO:0016887"
}